microbody [GO:0042579] (CC) Definition: Cytoplasmic organelles, spherical or oval in shape, that are bounded by a single membrane and contain oxidative enzymes, especially those utilizing hydrogen peroxide (H2O2). Sources: ISBN:0198506732 Relationships: is a type of intracellular membrane-bounded organelle [GO:0043231]; is part of cytoplasm [GO:0005737] Subtypes: peroxisome [GO:0005777], microbody membrane [GO:0031903], GO:0140266